positive regulation of mitochondrial translation [GO:0070131] (biological process) Also known as: positive regulation of mitochondrial protein anabolism, positive regulation of mitochondrial protein biosynthesis, positive regulation of mitochondrial protein formation, positive regulation of mitochondrial protein synthesis Definition: Any process that activates or increases the frequency, rate or extent of the chemical reactions and pathways resulting in the formation of proteins by the translation of mRNA in a mitochondrion. Sources: GOC:mah Subtypes: positive regulation of mitochondrial translation in response to stress [GO:0010892], positive regulation of mitochondrial translational initiation [GO:0070134] Relationships: is a type of positive regulation of translation [GO:0045727]; is a type of GO:0070129; positively regulates mitochondrial translation [GO:0032543]